mandelonitrile lyase activity [GO:0046593] (molecular function) Sources: EC:4.1.2.10 Relationships: is a type of aldehyde-lyase activity [GO:0016832] Also known as: hydroxynitrile lyase activity, (R)-oxynitrilase activity, D-alpha-hydroxynitrile lyase activity, D-oxynitrilase activity, mandelonitrile benzaldehyde-lyase (cyanide-forming), mandelonitrile benzaldehyde-lyase activity Definition: Catalysis of the reaction: mandelonitrile = cyanide + benzaldehyde.